{
  "gene_name": "Cyclic GMP-AMP synthase",
  "term_label": "activation of innate immune response",
  "gene_symbol": "CGAS",
  "gene": "UniProtKB:Q8N884",
  "term_id": "GO:0002218"
}